germ-line sex determination [GO:0018992] (biological process) Sources: GOC:ems Relationships: is a type of sex determination [GO:0007530]; BFO_0000050 multicellular organism development [GO:0007275] Definition: The determination of sex and sexual phenotype in an organism's germ line. Subtypes: female germ-line sex determination [GO:0019099], male germ-line sex determination [GO:0019100], hermaphrodite germ-line sex determination [GO:0040021]